regulation of vascular endothelial cell proliferation [GO:1905562] (biological process) References: PMID:23201774 Sources: GOC:BHF, GOC:BHF_telomere, GOC:TermGenie, GOC:nc, GO_REF:0000058 Definition: Any process that modulates the frequency, rate or extent of vascular endothelial cell proliferation. Relationships: is a type of regulation of endothelial cell proliferation [GO:0001936]; regulates vascular endothelial cell proliferation [GO:0101023] Subtypes: negative regulation of vascular endothelial cell proliferation [GO:1905563], positive regulation of vascular endothelial cell proliferation [GO:1905564]